L-xylulose reductase (NADPH) activity [GO:0050038] (molecular function) Relationships: is a type of oxidoreductase activity, acting on the CH-OH group of donors, NAD or NADP as acceptor [GO:0016616] Sources: RHEA:17025 Definition: Catalysis of the reaction: NADP+ + xylitol = L-xylulose + H+ + NADPH. Also known as: L-xylulose reductase activity